{
  "term_label": "Unknown cellular component",
  "term_id": "UNKNOWN:0003",
  "gene_name": "Tubulin polyglutamylase complex subunit 2",
  "gene": "UniProtKB:Q68CL5",
  "gene_symbol": "TPGS2"
}